{
  "gene": "UniProtKB:Q96AA8",
  "gene_symbol": "JAKMIP2",
  "term_id": "UNKNOWN:0002",
  "gene_name": "Janus kinase and microtubule-interacting protein 2",
  "term_label": "Unknown biological process"
}